{
  "term_label": "cytosol",
  "gene_name": "CBP80_20-dependent translation initiation factor",
  "term_id": "GO:0005829",
  "gene": "UniProtKB:O43310",
  "gene_symbol": "CTIF"
}